{
  "term_label": "chromatin organization",
  "gene_symbol": "RAD54L2",
  "gene_name": "Helicase ARIP4",
  "term_id": "GO:0006325",
  "gene": "UniProtKB:Q9Y4B4"
}